{
  "term_label": "exocytosis",
  "gene": "UniProtKB:P61266",
  "term_id": "GO:0006887",
  "gene_symbol": "STX1B",
  "gene_name": "Syntaxin-1B"
}